{
  "gene_symbol": "PDF",
  "term_label": "Unknown biological process",
  "term_id": "UNKNOWN:0002",
  "gene_name": "Peptide deformylase, mitochondrial",
  "gene": "UniProtKB:Q9HBH1"
}